{
  "term_label": "regulation of membrane potential",
  "gene_symbol": "PIEZO1",
  "term_id": "GO:0042391",
  "gene": "UniProtKB:Q92508",
  "gene_name": "Piezo-type mechanosensitive ion channel component 1"
}